{
  "gene_symbol": "FAM114A2",
  "term_id": "UNKNOWN:0001",
  "term_label": "Unknown molecular function",
  "gene_name": "Protein FAM114A2",
  "gene": "UniProtKB:Q9NRY5"
}